{
  "gene": "UniProtKB:Q9P1P5",
  "gene_name": "Trace amine-associated receptor 2",
  "term_id": "GO:0007186",
  "term_label": "G protein-coupled receptor signaling pathway",
  "gene_symbol": "TAAR2"
}